mitochondrial crista junction [GO:0044284] (cellular component) References: PMID:21944719, PMID:21987634, PMID:22009199 Sources: GOC:mcc Also known as: crista junction, cristae junction Relationships: is a type of organelle membrane contact site [GO:0044232]; is part of mitochondrial inner membrane [GO:0005743] Definition: A tubular structure of relatively uniform size that connects a mitochondrial crista to the mitochondrial inner boundary membrane.